{
  "gene_name": "von Willebrand factor A domain-containing protein 2",
  "gene_symbol": "VWA2",
  "term_label": "calcium-independent cell-matrix adhesion",
  "term_id": "GO:0007161",
  "gene": "UniProtKB:Q5GFL6"
}